{
  "gene": "UniProtKB:Q96EP0",
  "term_id": "GO:0097039",
  "term_label": "protein linear polyubiquitination",
  "gene_symbol": "RNF31",
  "gene_name": "E3 ubiquitin-protein ligase RNF31"
}